{
  "term_id": "GO:0070728",
  "term_label": "L-leucine binding",
  "gene_symbol": "SESN1",
  "gene": "UniProtKB:Q9Y6P5",
  "gene_name": "Sestrin-1"
}